{
  "gene_name": "Zinc finger protein 140",
  "gene_symbol": "ZNF140",
  "term_id": "GO:0000978",
  "term_label": "RNA polymerase II cis-regulatory region sequence-specific DNA binding",
  "gene": "UniProtKB:P52738"
}